aldose-1-phosphate nucleotidyltransferase activity [GO:0047347] (molecular function) Also known as: NDP-sugar phosphorylase activity, sugar-1-phosphate nucleotidyltransferase activity, NDP sugar phosphorylase activity, NDP-aldose phosphorylase activity, NDP:aldose-1-phosphate nucleotidyltransferase activity, NDP:alpha-D-aldose-1-phosphate nucleotidyltransferase activity, NDPaldose phosphorylase activity, glucose 1-phosphate inosityltransferase activity, nucleoside diphosphate sugar:orthophosphate nucleotidyltransferase activity, nucleoside diphosphosugar phosphorylase activity, sugar nucleotide phosphorylase activity, sugar phosphate nucleotidyltransferase activity Sources: EC:2.7.7.37, MetaCyc:2.7.7.37-RXN Relationships: is a type of GO:0016779 Definition: Catalysis of the reaction: aldose 1-phosphate + NDP = phosphate + NDP-aldose.